DnaB-DnaC complex [GO:1990100] (cellular component) Definition: A protein complex containing homohexameric DNA helicase DnaB, and the DNA helicase loader DnaC. The helicase loader DnaC delivers DnaB to the chromosomal origin (oriC). Note: DnaB and DnaC may be present in different ratios in different forms of the DnaB-DnaC complex, including a DnaB6-DnaC3 complex active at the oriC, and a DnaB6-DnaC6 complex. References: PMID:20129058 Sources: GOC:bhm Also known as: helicase-loading complex, DnaB6-DnaC3 complex, DnaB6-DnaC6 complex Relationships: is a type of protein-containing complex [GO:0032991]; BFO_0000050 GO:1990077; has part DnaB helicase complex [GO:1990161]